{
  "gene_symbol": "DESI2",
  "term_id": "UNKNOWN:0002",
  "gene_name": "Deubiquitinase DESI2",
  "gene": "UniProtKB:Q9BSY9",
  "term_label": "Unknown biological process"
}